photoprotection [GO:0010117] (biological process) Definition: Protection mechanism used by plants and cyanobacteria under conditions of excess energy absorption as a consequence of the light reactions of photosynthesis. Relationships: is a type of response to light stimulus [GO:0009416] References: PMID:30765616